{
  "term_id": "GO:0019373",
  "gene_name": "Cytochrome P450 2C9",
  "term_label": "epoxygenase P450 pathway",
  "gene_symbol": "CYP2C9",
  "gene": "UniProtKB:P11712"
}